{
  "gene_symbol": "RUVBL1",
  "term_label": "NuA4 histone acetyltransferase complex",
  "gene": "UniProtKB:Q9Y265",
  "gene_name": "RuvB-like 1",
  "term_id": "GO:0035267"
}